regulation of nitrate assimilation [GO:0090352] (biological process) Relationships: is a type of regulation of small molecule metabolic process [GO:0062012]; is a type of GO:1903314; regulates nitrate assimilation [GO:0042128] Sources: GOC:tb Definition: Any process that modulates the rate, frequency, or extent of the uptake, from the environment, of nitrates, inorganic or organic salts and esters of nitric acid and the subsequent reduction of nitrate ion to other, less highly oxidized, inorganic nitrogenous substances.